UDP-D-glucose:delphinidin 3-O-glucosyl-5-O-caffeoylglucoside -O-beta-D-glucosyltransferase activity [GO:0102816] (molecular function) Sources: EC:2.4.1.298, GOC:pz Definition: Catalysis of the reaction: UDP-alpha-D-glucose + delphinidin 3-O-glucosyl-5-O-caffeoylglucoside = H+ + delphinidin 3-O-glucosyl-5-O-(caffeoylglucoside-3'-O-glucoside) + UDP. Relationships: is a type of hexosyltransferase activity [GO:0016758]